lateral mesodermal cell fate commitment [GO:0048372] (biological process) Also known as: lateral mesoderm cell fate commitment, lateral plate mesoderm cell fate commitment, lateral plate mesodermal cell fate commitment Relationships: is_a mesodermal cell fate commitment [GO:0001710]; is part of lateral mesodermal cell differentiation [GO:0048371] Definition: The process in which a cell becomes committed to become a lateral mesoderm cell. Sources: GOC:jid